positive regulation of protein localization to cell leading edge [GO:1905873] (biological process) Also known as: positive regulation of protein localisation in cell leading edge, positive regulation of protein localisation to cell leading edge, positive regulation of protein localization in cell leading edge, up regulation of protein localisation in cell leading edge, up regulation of protein localisation to cell leading edge, up regulation of protein localization in cell leading edge, up regulation of protein localization to cell leading edge, up-regulation of protein localisation in cell leading edge, up-regulation of protein localisation to cell leading edge, up-regulation of protein localization in cell leading edge, up-regulation of protein localization to cell leading edge, upregulation of protein localisation in cell leading edge, upregulation of protein localisation to cell leading edge, upregulation of protein localization in cell leading edge, upregulation of protein localization to cell leading edge, activation of protein localisation in cell leading edge, activation of protein localisation to cell leading edge, activation of protein localization in cell leading edge, activation of protein localization to cell leading edge References: PMID:26324884 Sources: GOC:TermGenie, GO_REF:0000058 Relationships: is a type of positive regulation of protein localization [GO:1903829]; is a type of regulation of protein localization to cell leading edge [GO:1905871]; positively regulates protein localization to cell leading edge [GO:1902463] Definition: Any process that activates or increases the frequency, rate or extent of protein localization to cell leading edge.